{
  "gene_name": "Atrial natriuretic peptide receptor 1",
  "term_id": "GO:0004383",
  "gene": "UniProtKB:P16066",
  "term_label": "guanylate cyclase activity",
  "gene_symbol": "NPR1"
}